{
  "gene": "UniProtKB:Q2TAA2",
  "term_id": "UNKNOWN:0003",
  "term_label": "Unknown cellular component",
  "gene_name": "Isoamyl acetate-hydrolyzing esterase 1 homolog",
  "gene_symbol": "IAH1"
}